{
  "gene": "UniProtKB:Q8IVG9",
  "term_id": "UNKNOWN:0003",
  "gene_symbol": "MT-RNR2",
  "gene_name": "Humanin",
  "term_label": "Unknown cellular component"
}